{
  "gene_symbol": "APOA4",
  "gene": "UniProtKB:P06727",
  "term_label": "phospholipid efflux",
  "term_id": "GO:0033700",
  "gene_name": "Apolipoprotein A-IV"
}